{
  "term_id": "UNKNOWN:0002",
  "gene_name": "Putative uncharacterized protein encoded by LINC01356",
  "term_label": "Unknown biological process",
  "gene_symbol": "LINC01356",
  "gene": "UniProtKB:Q8N9X3"
}